{
  "term_label": "centrosome",
  "term_id": "GO:0005813",
  "gene_symbol": "CCDC77",
  "gene": "UniProtKB:Q9BR77",
  "gene_name": "Coiled-coil domain-containing protein 77"
}